membrane depolarization during action potential [GO:0086010] (biological process) Subtypes: membrane depolarization during cardiac muscle cell action potential [GO:0086012] Relationships: is a type of membrane depolarization [GO:0051899]; is part of action potential [GO:0001508] Regulation: regulated by regulation of membrane depolarization during action potential [GO:0098902] Definition: The process in which membrane potential changes in the depolarizing direction from the negative resting potential towards the positive membrane potential that will be the peak of the action potential. Sources: GOC:BHF, GOC:mtg_cardiac_conduct_nov11